{
  "gene": "UniProtKB:O96028",
  "term_label": "regulation of DNA-templated transcription",
  "term_id": "GO:0006355",
  "gene_symbol": "NSD2",
  "gene_name": "Histone-lysine N-methyltransferase NSD2"
}